{
  "term_label": "endocytosis",
  "gene_symbol": "ATP9B",
  "term_id": "GO:0006897",
  "gene_name": "Probable phospholipid-transporting ATPase IIB",
  "gene": "UniProtKB:O43861"
}